{
  "gene_name": "Peptidoglycan recognition protein 3",
  "term_label": "extracellular space",
  "term_id": "GO:0005615",
  "gene": "UniProtKB:Q96LB9",
  "gene_symbol": "PGLYRP3"
}